cement gland development [GO:0071570] (BP) Relationships: is a type of gland development [GO:0048732] Sources: GOC:bf Definition: The process whose specific outcome is the progression of the cement gland over time, from its formation to the mature structure. The cement gland is a simple mucus-secreting organ positioned at the anterior of amphibious embryos. The cement gland attaches the newly hatched embryo to a support before the hatchling can swim well or feed.